aerobic electron transport chain [GO:0019646] (biological process) Definition: A process in which a series of electron carriers operate together to transfer electrons from donors such as NADH and FADH2 to oxygen to generate a transmembrane electrochemical gradient. Relationships: is a type of aerobic respiration [GO:0009060]; is a type of GO:0022904; is part of oxidative phosphorylation [GO:0006119] Also known as: NADH-O2 electron transport, succinate-O2 electron transport, ubiquinone-8-O2 electron transport Subtypes: mitochondrial electron transport, NADH to ubiquinone [GO:0006120], mitochondrial electron transport, succinate to ubiquinone [GO:0006121], GO:0006122, mitochondrial electron transport, cytochrome c to oxygen [GO:0006123] Sources: GOC:ai, GOC:mtg_electron_transport